positive regulation of penetration hypha formation [GO:0075203] (biological process) Sources: GOC:pamgo_curators Definition: Any process that activates, maintains or increases the frequency, rate or extent of symbiont penetration hypha formation for entry into host. The host is defined as the larger of the organisms involved in a symbiotic interaction. Note: Note that this term should not be used to annotate gene products of the host. It should only be used to annotate those gene products from the symbiont involved in this process. Relationships: is a type of positive regulation of developmental process [GO:0051094]; is a type of regulation of penetration hypha formation [GO:0075202]; is a type of positive regulation by symbiont of entry into host [GO:0075294]; positively regulates penetration hypha formation [GO:0075201] Also known as: positive regulation of symbiont penetration hypha formation for entry into host